hydroxy-nicotine oxidase activity [GO:0019116] (molecular function) Subtypes: (R)-6-hydroxynicotine oxidase activity [GO:0018530], GO:0018531 References: PMID:16095622 Sources: GOC:jl Definition: Catalysis of the reaction: 6-hydroxynicotine + H2O + O2 = 1-(6-hydroxypyrid-3-yl)-4-(methylamino)butan-1-one + hydrogen peroxide. Relationships: is a type of oxidoreductase activity, acting on the CH-NH group of donors, oxygen as acceptor [GO:0016647]